{
  "term_label": "meiotic sister chromatid cohesion, centromeric",
  "gene": "UniProtKB:A0A087WXM9",
  "term_id": "GO:0051754",
  "gene_name": "Meiosis-specific kinetochore protein",
  "gene_symbol": "MEIKIN"
}